carbon fixation by 3-hydroxypropionate cycle [GO:0043427] (biological process) References: PMID:11418572, PMID:15838028 Sources: GOC:jl Also known as: 3-hydroxypropionate cycle, 3-hydroxypropionate pathway, hydroxypropionate cycle, hydroxypropionate pathway Relationships: is a type of carbon fixation [GO:0015977] Definition: An autotrophic carbon dioxide fixation pathway by which two molecules of carbon dioxide are fixed to form glyoxylate. Acetyl coenzyme A (acetyl-CoA) is assumed to be converted to malate, and two CO2 molecules are thereby fixed. Malyl-CoA is thought to be cleaved to acetyl-CoA, the starting molecule, and glyoxylate, the carbon fixation product.